negative regulation of myosin II filament organization [GO:1904900] (biological process) Definition: Any process that stops, prevents or reduces the frequency, rate or extent of myosin II filament organization. Also known as: down regulation of myosin II filament organisation, down regulation of myosin II filament organization, down-regulation of myosin II filament organisation, down-regulation of myosin II filament organization, downregulation of myosin II filament organisation, downregulation of myosin II filament organization, negative regulation of myosin II filament organisation, inhibition of myosin II filament organisation, inhibition of myosin II filament organization, down regulation of myosin II filament assembly or disassembly, down regulation of myosin II polymerization or depolymerization, down-regulation of myosin II filament assembly or disassembly, down-regulation of myosin II polymerization or depolymerization, downregulation of myosin II filament assembly or disassembly, downregulation of myosin II polymerization or depolymerization, inhibition of myosin II filament assembly or disassembly, inhibition of myosin II polymerization or depolymerization, negative regulation of myosin II filament assembly or disassembly, negative regulation of myosin II polymerization or depolymerization References: PMID:22761445 Sources: GOC:TermGenie, GO_REF:0000058 Relationships: is a type of GO:0043519; is a type of negative regulation of cytoskeleton organization [GO:0051494]; is a type of negative regulation of supramolecular fiber organization [GO:1902904]; negatively regulates myosin II filament organization [GO:0031038] Subtypes: negative regulation of myosin II filament assembly [GO:1905510]